establishment of protease localization to mast cell secretory granule [GO:0033372] (biological process) Also known as: establishment of protease localisation in mast cell secretory granule, establishment of protease localization in mast cell secretory granule Sources: GOC:mah Relationships: is_a establishment of protein localization to mast cell secretory granule [GO:0033369]; is part of protease localization to mast cell secretory granule [GO:0033368] Definition: The directed movement of a protease to a location within a secretory granule in a mast cell.